fatty-acyl-CoA biosynthetic process [GO:0046949] (biological process) Also known as: fatty acyl CoA biosynthetic process, fatty-acyl-CoA anabolism, fatty-acyl-CoA biosynthesis, fatty-acyl-CoA formation, fatty-acyl-CoA synthesis Subtypes: GO:0035338, butyryl-CoA biosynthetic process [GO:0044578], 2-methylbutanoyl-CoA(4-) biosynthetic process [GO:1902191], 2-methylbut-2-enoyl-CoA(4-) biosynthetic process [GO:1902194], isovaleryl-CoA(4-) biosynthetic process [GO:1902197], 3-methylbut-2-enoyl-CoA(4-) biosynthetic process [GO:1902200], propionyl-CoA biosynthetic process [GO:1902860] Definition: The chemical reactions and pathways resulting in the formation of a fatty-acyl-CoA, any derivative of coenzyme A in which the sulfhydryl group is in thiolester linkage with a fatty-acyl group. Relationships: is a type of fatty-acyl-CoA metabolic process [GO:0035337]; is a type of acyl-CoA biosynthetic process [GO:0071616]; is a type of fatty acid derivative biosynthetic process [GO:1901570] Sources: ISBN:0198506732